{
  "gene": "UniProtKB:Q96P31",
  "gene_name": "Fc receptor-like protein 3",
  "term_label": "cell surface receptor signaling pathway",
  "term_id": "GO:0007166",
  "gene_symbol": "FCRL3"
}